{
  "gene": "UniProtKB:Q9UP95",
  "gene_name": "Solute carrier family 12 member 4",
  "term_id": "GO:0055064",
  "term_label": "chloride ion homeostasis",
  "gene_symbol": "SLC12A4"
}